{
  "gene_symbol": "SPRY1",
  "gene": "UniProtKB:O43609",
  "gene_name": "Protein sprouty homolog 1",
  "term_id": "GO:0040037",
  "term_label": "negative regulation of fibroblast growth factor receptor signaling pathway"
}